{
  "gene_symbol": "KNG1",
  "term_label": "negative regulation of blood coagulation",
  "gene_name": "Kininogen-1",
  "gene": "UniProtKB:P01042",
  "term_id": "GO:0030195"
}